detection of misfolded protein [GO:0002236] (biological process) References: PMID:15226511 Sources: GOC:add Relationships: is a type of detection of chemical stimulus [GO:0009593]; is a type of response to misfolded protein [GO:0051788] Definition: The series of events in which a misfolded protein stimulus is received and converted into a molecular signal.